{
  "gene_symbol": "MMP9",
  "gene": "UniProtKB:P14780",
  "term_id": "GO:0030574",
  "term_label": "collagen catabolic process",
  "gene_name": "Matrix metalloproteinase-9"
}